{
  "gene_name": "Zinc finger protein 296",
  "term_id": "GO:0005634",
  "term_label": "nucleus",
  "gene": "UniProtKB:Q8WUU4",
  "gene_symbol": "ZNF296"
}